{
  "gene_name": "tRNA-splicing endonuclease subunit Sen2",
  "term_label": "tRNA-intron endonuclease complex",
  "gene": "UniProtKB:Q8NCE0",
  "term_id": "GO:0000214",
  "gene_symbol": "TSEN2"
}